{
  "gene_symbol": "MRGPRE",
  "term_label": "plasma membrane",
  "term_id": "GO:0005886",
  "gene": "UniProtKB:Q86SM8",
  "gene_name": "Mas-related G-protein coupled receptor member E"
}